N-acylethanolamine metabolic process [GO:0070291] (BP) Definition: The chemical reactions and pathways involving N-acylethanolamines. An N-acylethanolamine is an ethanolamine substituted at nitrogen by an acyl group. References: PMID:14634025, PMID:15878693 Sources: CHEBI:52640, GOC:elh Relationships: is_a primary alcohol metabolic process [GO:0034308] Also known as: N-acylethanolamine metabolism, NAE metabolic process, NAE metabolism